piccolo-bassoon transport vesicle [GO:1990257] (cellular component) Definition: A cytoplasmic dense-core vesicle that transports a range of proteins including piccolo, bassoon, N-cadherin and syntaxin. The transported proteins may be associated with the external side of the vesicle, rather than being contained within the vesicle, therefore forming an aggregate of vesicle and proteins. Piccolo-bassoon transport vesicles (or PTVs) range in size from approximately 80 nm in diameter for dense core vesicles to 130 nm by 220 nm in area for aggregates. They are packaged via the trans-Golgi network before being transported through the axon. References: PMID:21569270 Sources: GOC:dr Also known as: PTV Relationships: is a type of GO:0030133